2-(3-amino-3-carboxypropyl)histidine synthase activity [GO:0090560] (molecular function) References: PMID:15485916 Sources: GOC:pde, RHEA:36783 Relationships: is a type of GO:0016765 Definition: Catalysis of the reaction S-adenosyl-L-methionine + L-histidine-[translation elongation factor 2] = S-methyl-5-thioadenosine + 2-[(3S)-3-amino-3-carboxypropyl]-L-histidine-[translation elongation factor 2].